protein desuccinylation [GO:0036048] (biological process) Subtypes: peptidyl-lysine desuccinylation [GO:0036049] References: PMID:22076378 Sources: GOC:sp Relationships: is a type of GO:0035601 Definition: The removal of a succinyl group (CO-CH2-CH2-CO) from a residue in a peptide or protein.